{
  "gene_name": "von Willebrand factor D and EGF domain-containing protein",
  "term_label": "signaling receptor binding",
  "gene": "UniProtKB:Q8N2E2",
  "gene_symbol": "VWDE",
  "term_id": "GO:0005102"
}